{
  "gene_name": "Ferroptosis suppressor protein 1",
  "gene_symbol": "AIFM2",
  "gene": "UniProtKB:Q9BRQ8",
  "term_label": "negative regulation of ferroptosis",
  "term_id": "GO:0110076"
}